RNA import into nucleus [GO:0006404] (biological process) Definition: The import of RNA from the cytoplasm to the nucleus. Sources: GOC:ma Regulation: regulated by GO:0046828; negatively regulated by GO:0046829; RO_0002213 by positive regulation of RNA import into nucleus [GO:0046830] Subtypes: tRNA import into nucleus [GO:0035719], snRNA import into nucleus [GO:0061015] Also known as: RNA import into cell nucleus, RNA transport from cytoplasm to nucleus, RNA-nucleus import Relationships: is a type of RNA transport [GO:0050658]; is a type of import into nucleus [GO:0051170]